{
  "term_id": "GO:0005737",
  "term_label": "cytoplasm",
  "gene_name": "Cytochrome P450 2F1",
  "gene_symbol": "CYP2F1",
  "gene": "UniProtKB:P24903"
}